{
  "term_id": "GO:0005096",
  "gene": "UniProtKB:O43566",
  "term_label": "GTPase activator activity",
  "gene_symbol": "RGS14",
  "gene_name": "Regulator of G-protein signaling 14"
}